negative regulation of smooth muscle cell apoptotic process [GO:0034392] (biological process) Definition: Any process that stops, prevents, or reduces the frequency, rate, or extent of smooth muscle cell apoptotic process. Subtypes: GO:1905460 Sources: GOC:BHF, GOC:mtg_apoptosis, GOC:rl Also known as: down regulation of smooth muscle cell apoptosis, down-regulation of smooth muscle cell apoptosis, downregulation of smooth muscle cell apoptosis, negative regulation of SMC apoptosis, inhibition of smooth muscle cell apoptosis, negative regulation of smooth muscle cell apoptosis Relationships: is a type of negative regulation of muscle cell apoptotic process [GO:0010656]; is a type of regulation of smooth muscle cell apoptotic process [GO:0034391]; RO_0002212 smooth muscle cell apoptotic process [GO:0034390]